{
  "gene": "UniProtKB:Q8N5Q1",
  "term_label": "Unknown cellular component",
  "gene_name": "Golgi-associated RAB2 interactor protein 5B",
  "gene_symbol": "GARIN5B",
  "term_id": "UNKNOWN:0003"
}